{
  "term_label": "calcium-dependent phospholipid binding",
  "gene_symbol": "ANXA2P2",
  "term_id": "GO:0005544",
  "gene_name": "Putative annexin A2-like protein",
  "gene": "UniProtKB:A6NMY6"
}